negative regulation of protein linear polyubiquitination [GO:1902529] (biological process) References: PMID:21931591 Sources: GOC:TermGenie Definition: Any process that stops, prevents or reduces the frequency, rate or extent of protein linear polyubiquitination. Relationships: is a type of regulation of protein linear polyubiquitination [GO:1902528]; is a type of GO:1902915; negatively regulates GO:0097039 Also known as: down regulation of protein linear polyubiquitination, down-regulation of protein linear polyubiquitination, downregulation of protein linear polyubiquitination, down regulation of M1 linkage, down-regulation of M1 linkage, downregulation of M1 linkage, inhibition of M1 linkage, inhibition of protein linear polyubiquitination, negative regulation of M1 linkage